{
  "term_id": "GO:0005739",
  "gene_name": "T-cell activation inhibitor, mitochondrial",
  "term_label": "mitochondrion",
  "gene_symbol": "TCAIM",
  "gene": "UniProtKB:Q8N3R3"
}